ryanodine receptor complex [GO:1990425] (cellular component) Definition: A voltage-gated calcium-release channel complex of the sarcoplasmic or endoplasmic reticulum. It plays an important role in the excitation-contraction (E-C) coupling of muscle cells. RyR comprises a family of ryanodine receptors, widely expressed throughout the animal kingdom. Also known as: RyR Note: An example of this is RyR1 in rabbit (P11716) in PMID:2550460 (inferred from electron microscopy). Relationships: is a type of voltage-gated calcium channel complex [GO:0005891]; is a type of GO:0140534; BFO_0000050 sarcoplasmic reticulum membrane [GO:0033017] References: PMID:22822064 Sources: GOC:ame